lysosomal transport [GO:0007041] (biological process) Relationships: is a type of GO:0007034 Definition: The directed movement of substances into, out of or within a lysosome. Subtypes: GO:0006622, endosome to lysosome transport [GO:0008333], lysosome to ER cholesterol transport [GO:0090120], Golgi to lysosome transport [GO:0090160], GO:0099074, zinc ion import into lysosome [GO:0140916], purine nucleotide import into lysosome [GO:0141013], transmembrane transport from lysosomal lumen to cytosol [GO:0170063], GO:1902774 Sources: GOC:ai